{
  "gene_symbol": "SUPV3L1",
  "gene": "UniProtKB:Q8IYB8",
  "term_label": "Unknown molecular function",
  "gene_name": "ATP-dependent RNA helicase SUPV3L1, mitochondrial",
  "term_id": "UNKNOWN:0001"
}